{
  "gene": "UniProtKB:P0DPF6",
  "term_label": "Unknown cellular component",
  "gene_symbol": "CDRT15P3",
  "term_id": "UNKNOWN:0003",
  "gene_name": "Putative uncharacterized protein CDRT15P3"
}